strictosidine beta-glucosidase activity [GO:0050422] (molecular function) Also known as: strictosidine b-glucosidase activity, strictosidine beta-D-glucohydrolase activity Sources: EC:3.2.1.105, RHEA:12917 Relationships: is a type of beta-glucosidase activity [GO:0008422] Definition: Catalysis of the reaction: 3alpha(S)-strictosidine + H2O = D-glucose + strictosidine aglycone.